{
  "term_id": "GO:0048812",
  "gene_symbol": "MNX1",
  "term_label": "neuron projection morphogenesis",
  "gene": "UniProtKB:P50219",
  "gene_name": "Motor neuron and pancreas homeobox protein 1"
}